{
  "term_id": "GO:0006552",
  "gene": "UniProtKB:P26440",
  "gene_name": "Isovaleryl-CoA dehydrogenase, mitochondrial",
  "term_label": "L-leucine catabolic process",
  "gene_symbol": "IVD"
}